parallel fiber [GO:1990032] (cellular component) Sources: ISBN:0195159551, NIF_Subcellular:nlx_330 Definition: A parallel fiber results from the bifurcation of a cerebellar granule cell axon in the molecular layer into two diametrically opposed branches, that are oriented parallel to the long axis of the folium. Relationships: is a type of axon [GO:0030424]